{
  "term_id": "GO:0030881",
  "term_label": "beta-2-microglobulin binding",
  "gene_symbol": "HLA-H",
  "gene": "UniProtKB:P01893",
  "gene_name": "Putative HLA class I histocompatibility antigen, alpha chain H"
}